{
  "term_id": "GO:0042424",
  "term_label": "catecholamine catabolic process",
  "gene_name": "Catechol O-methyltransferase",
  "gene": "UniProtKB:P21964",
  "gene_symbol": "COMT"
}